negative regulation of apoptotic process in bone marrow cell [GO:0071866] (biological process) Relationships: is a type of GO:0043066; is a type of regulation of apoptotic process in bone marrow cell [GO:0071865]; negatively regulates GO:0071839 Definition: Any process that stops, prevents, or reduces the frequency, rate or extent of the occurrence or rate of cell death by apoptotic process in the bone marrow. Also known as: down regulation of apoptosis in bone marrow, down-regulation of apoptosis in bone marrow, downregulation of apoptosis in bone marrow, negative regulation of apoptotic process in bone marrow, negative regulation of bone marrow cell apoptosis, negative regulation of bone marrow cell programmed cell death by apoptosis, negative regulation of killing of bone marrow cells, negative regulation of programmed cell death of bone marrow cells by apoptosis, negative regulation of programmed cell death, bone marrow cells, inhibition of apoptosis in bone marrow, negative regulation of apoptosis in bone marrow References: PMID:17063141 Sources: GOC:mah, GOC:mtg_apoptosis, GOC:yaf